{
  "gene_name": "Protein S100-A5",
  "gene_symbol": "S100A5",
  "term_label": "Unknown biological process",
  "gene": "UniProtKB:P33763",
  "term_id": "UNKNOWN:0002"
}